{
  "gene_name": "Protein SPT2 homolog",
  "gene": "UniProtKB:Q68D10",
  "term_label": "histone binding",
  "term_id": "GO:0042393",
  "gene_symbol": "SPTY2D1"
}